{
  "term_label": "cytosol",
  "gene_symbol": "USP17L18",
  "term_id": "GO:0005829",
  "gene": "UniProtKB:D6R9N7",
  "gene_name": "Ubiquitin carboxyl-terminal hydrolase 17-like protein 18"
}